{
  "gene": "UniProtKB:Q969N4",
  "term_label": "plasma membrane",
  "gene_name": "Trace amine-associated receptor 8",
  "term_id": "GO:0005886",
  "gene_symbol": "TAAR8"
}